{
  "term_id": "UNKNOWN:0001",
  "gene": "UniProtKB:Q9P227",
  "gene_name": "Rho GTPase-activating protein 23",
  "gene_symbol": "ARHGAP23",
  "term_label": "Unknown molecular function"
}